{
  "term_id": "GO:0007265",
  "term_label": "Ras protein signal transduction",
  "gene_symbol": "RIT2",
  "gene": "UniProtKB:Q99578",
  "gene_name": "GTP-binding protein Rit2"
}